{
  "term_label": "Unknown biological process",
  "gene_symbol": "ZMAT5",
  "gene": "UniProtKB:Q9UDW3",
  "gene_name": "Zinc finger matrin-type protein 5",
  "term_id": "UNKNOWN:0002"
}